positive regulation of smooth muscle cell chemotaxis [GO:0071673] (biological process) Definition: Any process that activates or increases the frequency, rate, or extent of smooth muscle cell chemotaxis. Sources: GOC:mah Also known as: up regulation of smooth muscle cell chemotaxis, up-regulation of smooth muscle cell chemotaxis, upregulation of smooth muscle cell chemotaxis, activation of smooth muscle cell chemotaxis, stimulation of smooth muscle cell chemotaxis Relationships: is a type of GO:0014911; is a type of positive regulation of chemotaxis [GO:0050921]; is a type of regulation of smooth muscle cell chemotaxis [GO:0071671]; positively regulates smooth muscle cell chemotaxis [GO:0071670]